trichome papilla [GO:0090705] (cellular component) Relationships: is a type of plant cell papilla [GO:0090395] Note: Part of trichome cell (PO:0008030). References: PMID:24014871 Sources: GOC:tb Definition: A plant cell papilla that is part of a trichome cell.